{
  "gene_name": "Interleukin-34",
  "gene_symbol": "IL34",
  "term_id": "GO:0045651",
  "gene": "UniProtKB:Q6ZMJ4",
  "term_label": "positive regulation of macrophage differentiation"
}